{
  "term_id": "GO:0032454",
  "gene_name": "Lysine-specific demethylase 3B",
  "term_label": "histone H3K9 demethylase activity",
  "gene": "UniProtKB:Q7LBC6",
  "gene_symbol": "KDM3B"
}